{
  "term_label": "DNA-binding transcription factor activity",
  "gene_symbol": "ZBTB48",
  "term_id": "GO:0003700",
  "gene_name": "Telomere zinc finger-associated protein",
  "gene": "UniProtKB:P10074"
}